{
  "term_label": "plus-end-directed microtubule motor activity",
  "gene": "UniProtKB:Q9P2E2",
  "gene_symbol": "KIF17",
  "term_id": "GO:0008574",
  "gene_name": "Kinesin-like protein KIF17"
}